{
  "gene_name": "DNA mismatch repair protein Msh6",
  "gene": "UniProtKB:P52701",
  "term_label": "mismatch repair",
  "gene_symbol": "MSH6",
  "term_id": "GO:0006298"
}